{
  "term_label": "cysteine-type deubiquitinase activity",
  "gene": "UniProtKB:Q9P2H5",
  "gene_name": "Ubiquitin carboxyl-terminal hydrolase 35",
  "gene_symbol": "USP35",
  "term_id": "GO:0004843"
}